{
  "term_id": "GO:0034728",
  "gene_name": "Chromodomain-helicase-DNA-binding protein 2",
  "gene": "UniProtKB:O14647",
  "term_label": "nucleosome organization",
  "gene_symbol": "CHD2"
}